protein localization to adherens junction [GO:0071896] (biological process) Definition: Any process in which a protein is transported to, and/or maintained at the adherens junction. References: PMID:26412237 Sources: GOC:BHF, GOC:aruk, GOC:bc, GOC:mah Also known as: protein localisation in adherens junction, protein localisation in cell-cell adherens junction, protein localisation to adherens junction, protein localisation to cell-cell adherens junction, protein localization in adherens junction, protein localization in cell-cell adherens junction, protein localization to cell-cell adherens junction Relationships: is a type of protein localization to cell-cell junction [GO:0150105] Regulation: regulated by regulation of protein localization to adherens junction [GO:1904702]; negatively regulated by GO:1904703; positively regulated by positive regulation of protein localization to adherens junction [GO:1904704]